{
  "term_id": "GO:0010043",
  "gene": "UniProtKB:Q99726",
  "term_label": "response to zinc ion",
  "gene_name": "Probable proton-coupled zinc antiporter SLC30A3",
  "gene_symbol": "SLC30A3"
}